non-kinase phorbol ester receptor activity [GO:0001566] (MF) Definition: Combining with a phorbol ester and transmitting the signal by a mechanism independent of kinase activity. Relationships: is a type of GO:0001565 References: PMID:10506570